{
  "gene": "UniProtKB:Q99584",
  "term_label": "extracellular space",
  "term_id": "GO:0005615",
  "gene_symbol": "S100A13",
  "gene_name": "Protein S100-A13"
}